{
  "gene": "UniProtKB:Q8NGX5",
  "gene_name": "Olfactory receptor 10K1",
  "gene_symbol": "OR10K1",
  "term_id": "GO:0005549",
  "term_label": "odorant binding"
}